{
  "term_label": "base-excision repair",
  "gene_symbol": "MPG",
  "gene_name": "DNA-3-methyladenine glycosylase",
  "gene": "UniProtKB:P29372",
  "term_id": "GO:0006284"
}